positive regulation of horizontal cell localization [GO:1902874] (biological process) Definition: Any process that activates or increases the frequency, rate or extent of horizontal cell localization. Also known as: positive regulation of horizontal cell localisation, positive regulation of horizontal cell positioning, positive regulation of laminar positioning of retinal horizontal cell, positive regulation of retinal horizontal cell positioning, up regulation of horizontal cell localisation, up regulation of horizontal cell localization, up regulation of horizontal cell positioning, up regulation of laminar positioning of retinal horizontal cell, up regulation of retinal horizontal cell positioning, up-regulation of horizontal cell localisation, up-regulation of horizontal cell localization, up-regulation of horizontal cell positioning, up-regulation of laminar positioning of retinal horizontal cell, up-regulation of retinal horizontal cell positioning, upregulation of horizontal cell localisation, upregulation of horizontal cell localization, upregulation of horizontal cell positioning, upregulation of laminar positioning of retinal horizontal cell, upregulation of retinal horizontal cell positioning, activation of horizontal cell localisation, activation of horizontal cell localization, activation of horizontal cell positioning, activation of laminar positioning of retinal horizontal cell, activation of retinal horizontal cell positioning Relationships: is a type of positive regulation of cellular process [GO:0048522]; is a type of regulation of horizontal cell localization [GO:1902872]; positively regulates horizontal cell localization [GO:0035852] References: PMID:16872597 Sources: GOC:TermGenie, GOC:mr, GO_REF:0000058